{
  "gene_symbol": "PM20D1",
  "gene_name": "N-fatty-acyl-amino acid synthase_hydrolase PM20D1",
  "gene": "UniProtKB:Q6GTS8",
  "term_label": "amide biosynthetic process",
  "term_id": "GO:0043604"
}